{
  "gene_symbol": "C11orf54",
  "gene_name": "Ester hydrolase C11orf54",
  "term_id": "GO:0008270",
  "gene": "UniProtKB:Q9H0W9",
  "term_label": "zinc ion binding"
}